{
  "gene": "UniProtKB:A5D8V6",
  "term_id": "GO:0006612",
  "gene_symbol": "VPS37C",
  "gene_name": "Vacuolar protein sorting-associated protein 37C",
  "term_label": "protein targeting to membrane"
}